carboxyl-O-methyltransferase activity [GO:0010340] (molecular function) References: PMID:17220201 Subtypes: gibberellin carboxyl-O-methyltransferase activity [GO:0010341], protein carboxyl O-methyltransferase activity [GO:0051998] Definition: Catalysis of the transfer of a methyl group to the carboxyl group of an acceptor molecule to form a methyl ester. Relationships: is_a O-methyltransferase activity [GO:0008171]